{
  "gene_name": "Protein canopy homolog 2",
  "gene": "UniProtKB:Q9Y2B0",
  "term_label": "Unknown biological process",
  "term_id": "UNKNOWN:0002",
  "gene_symbol": "CNPY2"
}